{
  "gene": "UniProtKB:Q13519",
  "term_label": "opioid receptor binding",
  "term_id": "GO:0031628",
  "gene_name": "Prepronociceptin",
  "gene_symbol": "PNOC"
}